{
  "gene_symbol": "PRAME",
  "term_label": "cytoplasm",
  "term_id": "GO:0005737",
  "gene_name": "Melanoma antigen preferentially expressed in tumors",
  "gene": "UniProtKB:P78395"
}